purine nucleoside transmembrane transporter activity [GO:0015211] (molecular function) Sources: GOC:ai Definition: Enables the transfer of a purine nucleoside, a purine base covalently bonded to a ribose or deoxyribose sugar, from one side of a membrane to the other. Relationships: is a type of nucleoside transmembrane transporter activity [GO:0005337]; is part of purine nucleoside transmembrane transport [GO:0015860] Subtypes: xanthosine transmembrane transporter activity [GO:0015553], S-adenosyl-L-methionine:S-adenosyl-L-homocysteine antiporter activity [GO:0180003]